autoinducer AI-2 transmembrane transport [GO:1905887] (biological process) Definition: The process in which (2R,4S)-2-methyltetrahydrofuran-2,3,3,4-tetrol (autoinducer AI-2) is transported across a membrane. AI-2 is produced by prokaryotes and is believed to play a role in quorum sensing. References: PMID:15601708 Sources: GOC:TermGenie, GO_REF:0000069 Also known as: (2R,4S)-2-methyltetrahydrofuran-2,3,3,4-tetrol transmembrane transport, AI-2 transmembrane transport, autoinducer 2 transmembrane transport Relationships: is a type of polyol transmembrane transport [GO:0015791]